{
  "term_id": "GO:0045095",
  "gene": "UniProtKB:P02538",
  "gene_symbol": "KRT6A",
  "term_label": "keratin filament",
  "gene_name": "Keratin, type II cytoskeletal 6A"
}